{
  "term_label": "Ras protein signal transduction",
  "gene_symbol": "RASSF1",
  "gene": "UniProtKB:Q9NS23",
  "gene_name": "Ras association domain-containing protein 1",
  "term_id": "GO:0007265"
}